{
  "gene_name": "C-terminal-binding protein 1",
  "term_id": "GO:0003714",
  "term_label": "transcription corepressor activity",
  "gene": "UniProtKB:Q13363",
  "gene_symbol": "CTBP1"
}